{
  "gene": "UniProtKB:Q5T1C6",
  "gene_symbol": "THEM4",
  "term_label": "long-chain fatty acyl-CoA hydrolase activity",
  "gene_name": "Acyl-coenzyme A thioesterase THEM4",
  "term_id": "GO:0052816"
}